{
  "term_id": "UNKNOWN:0002",
  "gene_symbol": "CYP4Z2P",
  "gene_name": "Putative inactive cytochrome P450 family member 4Z2",
  "gene": "UniProtKB:Q8N1L4",
  "term_label": "Unknown biological process"
}